{
  "term_label": "Unknown cellular component",
  "gene_symbol": "LGALS13",
  "gene_name": "Galactoside-binding soluble lectin 13",
  "gene": "UniProtKB:Q9UHV8",
  "term_id": "UNKNOWN:0003"
}